{
  "gene_symbol": "TMOD1",
  "term_id": "GO:0030239",
  "gene_name": "Tropomodulin-1",
  "term_label": "myofibril assembly",
  "gene": "UniProtKB:P28289"
}